ADP-specific glucokinase activity [GO:0043843] (molecular function) Definition: Catalysis of the reaction: ADP + D-glucose = AMP + D-glucose 6-phosphate. Sources: EC:2.7.1.147 Relationships: is a type of kinase activity [GO:0016301]; is a type of GO:0016773 Also known as: ADP-dependent glucokinase activity, ADP:D-glucose 6-phosphotransferase activity